germ-band shortening [GO:0007390] (biological process) Relationships: is a type of embryonic morphogenesis [GO:0048598]; BFO_0000050 embryonic development via the syncytial blastoderm [GO:0001700] References: PMID:12147138 Sources: GOC:bf Definition: The spreading of the amnioserosa from its compressed state to cover the whole of the dorsal surface. Initiating in the thorax and spreading posteriorly, it is accompanied by the transition from a parasegmental to segmental division of the embryo. Also known as: germ-band retraction